{
  "term_id": "UNKNOWN:0002",
  "gene": "UniProtKB:Q6PK04",
  "gene_symbol": "CCDC137",
  "gene_name": "Coiled-coil domain-containing protein 137",
  "term_label": "Unknown biological process"
}